apolipoprotein A-I receptor binding [GO:0034191] (molecular function) Note: Note that this term is to be used only to annotate gene products that bind to lipid-free APOA1. For receptors that bind lipid-associated apolipoproteins (plasma lipoprotein particles), consider annotating to 'lipoprotein receptor activity ; GO:0030228' or its child terms. Definition: Binding to an apolipoprotein A-I receptor. Sources: GOC:BHF, GOC:rl Relationships: is a type of apolipoprotein receptor binding [GO:0034190]